{
  "gene": "UniProtKB:Q8N9W8",
  "term_label": "Unknown biological process",
  "term_id": "UNKNOWN:0002",
  "gene_symbol": "GARIN2",
  "gene_name": "Golgi-associated RAB2 interactor protein 2"
}